{
  "term_label": "negative regulation of apoptotic process",
  "gene_symbol": "SPHK1",
  "term_id": "GO:0043066",
  "gene": "UniProtKB:Q9NYA1",
  "gene_name": "Sphingosine kinase 1"
}